thiamine binding [GO:0030975] (molecular function) Also known as: thiamin binding, vitamin B1 binding Relationships: is_a vitamin binding [GO:0019842]; is a type of GO:0043169; is a type of GO:0043178; is a type of heterocyclic compound binding [GO:1901363]; is a type of GO:1901681 Definition: Binding to thiamine (vitamin B1), a water soluble vitamin present in fresh vegetables and meats, especially liver. Sources: GOC:mlg